gibberellin 3-beta-dioxygenase activity [GO:0016707] (molecular function) References: PMID:32652020 Sources: EC:1.14.11.15 Relationships: is a type of 2-oxoglutarate-dependent dioxygenase activity [GO:0016706] Also known as: (gibberellin-20),2-oxoglutarate:oxygen oxidoreductase (3beta-hydroxylating), (gibberrellin-20),2-oxoglutarate: oxygen oxidoreductase (3beta-hydroxylating), gibberellin 3-beta-hydroxylase activity, gibberellin 3beta-dioxygenase activity, gibberellin 3beta-hydroxylase activity Definition: Catalysis of the reaction: a gibberellin + 2-oxoglutarate + O2 = a 3-beta-hydroxy-gibberellin + succinate + CO2.